{
  "term_label": "regulation of transcription by RNA polymerase II",
  "term_id": "GO:0006357",
  "gene": "UniProtKB:P31274",
  "gene_symbol": "HOXC9",
  "gene_name": "Homeobox protein Hox-C9"
}